regulation of intermediate filament polymerization or depolymerization [GO:0045108] (biological process) Relationships: is a type of regulation of cellular component organization [GO:0051128]; regulates intermediate filament polymerization or depolymerization [GO:0045105] Definition: Any process that modulates the frequency, rate or extent of the assembly or disassembly of intermediate filaments by the addition or removal of monomers from a filament; this usually occurs through the opposing action of kinases and phosphatases. Subtypes: GO:0030839, regulation of intermediate filament depolymerization [GO:0030842] Sources: ISBN:0716731363